negative regulation of sorocarp stalk cell differentiation [GO:0031286] (biological process) Definition: Any process that stops, prevents, or reduces the frequency, rate or extent of sorocarp stalk cell differentiation. An example of this process is found in Dictyostelium discoideum. References: PMID:4338436 Sources: GOC:kp, GOC:mtg_sensu Also known as: down regulation of stalk cell differentiation, down-regulation of stalk cell differentiation, downregulation of stalk cell differentiation, negative regulation of stalk cell differentiation, inhibition of stalk cell differentiation Relationships: is a type of regulation of sorocarp stalk cell differentiation [GO:0031285]; is a type of negative regulation of response to nutrient levels [GO:0032108]; is a type of negative regulation of cell differentiation [GO:0045596]; is a type of negative regulation of spore-bearing organ development [GO:0075262]; negatively regulates sorocarp stalk cell differentiation [GO:0031149]